{
  "term_id": "UNKNOWN:0001",
  "term_label": "Unknown molecular function",
  "gene_symbol": "TRMT6",
  "gene": "UniProtKB:Q9UJA5",
  "gene_name": "tRNA (adenine(58)-N(1))-methyltransferase non-catalytic subunit TRM6"
}